{
  "gene_symbol": "C21orf62-AS1",
  "term_label": "Unknown cellular component",
  "gene_name": "Putative uncharacterized protein C21orf62-AS1",
  "term_id": "UNKNOWN:0003",
  "gene": "UniProtKB:Q17RA5"
}